{
  "gene": "UniProtKB:P07203",
  "gene_symbol": "GPX1",
  "term_id": "GO:0005829",
  "gene_name": "Glutathione peroxidase 1",
  "term_label": "cytosol"
}